{
  "term_id": "UNKNOWN:0003",
  "gene_name": "RNA ligase 1",
  "gene": "UniProtKB:Q8N999",
  "gene_symbol": "RLIG1",
  "term_label": "Unknown cellular component"
}